tryptophan 5-monooxygenase activity [GO:0004510] (molecular function) Definition: Catalysis of the reaction: L-tryptophan + tetrahydrobiopterin + O2 = 5-hydroxy-L-tryptophan + 4-alpha-hydroxytetrahydrobiopterin + H2O. Sources: EC:1.14.16.4 Also known as: L-tryptophan hydroxylase activity, L-tryptophan,tetrahydrobiopterin:oxygen oxidoreductase (5-hydroxylating), indoleacetic acid-5-hydroxylase activity, tryptophan 5-hydroxylase activity, tryptophan hydroxylase activity Relationships: is a type of oxidoreductase activity, acting on paired donors, with incorporation or reduction of molecular oxygen, reduced pteridine as one donor, and incorporation of one atom of oxygen [GO:0016714] Regulation: positively regulated by GO:0016483